{
  "gene_symbol": "IGHD1-1",
  "term_label": "Unknown biological process",
  "gene_name": "Immunoglobulin heavy diversity 1-1",
  "gene": "UniProtKB:P0DOY5",
  "term_id": "UNKNOWN:0002"
}